{
  "term_id": "GO:0034364",
  "gene": "UniProtKB:P06727",
  "gene_symbol": "APOA4",
  "gene_name": "Apolipoprotein A-IV",
  "term_label": "high-density lipoprotein particle"
}